{
  "gene_symbol": "ZNF26",
  "gene_name": "Zinc finger protein 26",
  "term_id": "UNKNOWN:0003",
  "term_label": "Unknown cellular component",
  "gene": "UniProtKB:P17031"
}